{
  "gene_name": "GPI mannosyltransferase 1",
  "term_label": "glycosylphosphatidylinositol-mannosyltransferase I complex",
  "term_id": "GO:1990529",
  "gene": "UniProtKB:Q9H3S5",
  "gene_symbol": "PIGM"
}